{
  "gene_name": "Methyl-CpG-binding domain protein 2",
  "term_id": "GO:0005634",
  "gene_symbol": "MBD2",
  "gene": "UniProtKB:Q9UBB5",
  "term_label": "nucleus"
}